{
  "gene_symbol": "CAV3",
  "term_label": "caveola",
  "term_id": "GO:0005901",
  "gene": "UniProtKB:P56539",
  "gene_name": "Caveolin-3"
}